{
  "term_id": "UNKNOWN:0001",
  "gene_name": "Putative WAS protein family homolog 3",
  "term_label": "Unknown molecular function",
  "gene_symbol": "WASH3P",
  "gene": "UniProtKB:C4AMC7"
}